{
  "term_label": "cytoplasmic translation",
  "gene_symbol": "RPL22L1",
  "term_id": "GO:0002181",
  "gene_name": "Ribosomal protein eL22-like",
  "gene": "UniProtKB:Q6P5R6"
}